ribosome translocase activity [GO:0180054] (MF) References: PMID:19173642 Relationships: is a type of GTPase motor activity [GO:0061791] Definition: A motor activity that generates movement of a ribosome one codon forward along the mRNA, driven by GTP hydrolysis.